ABC-type polyamine transporter activity [GO:0015417] (molecular function) Also known as: polyamine porter activity, ATPase-coupled spermidine transmembrane transporter activity, polyamine ABC transporter, polyamine-importing ATPase activity, spermidine porter activity, spermidine-importing ATPase activity, ATP-dependent polyamine transmembrane transporter activity, ATPase-coupled polyamine transmembrane transporter activity, polyamine-transporting ATPase activity Sources: RHEA:29999 Relationships: is a type of polyamine transmembrane transporter activity [GO:0015203]; is a type of GO:0140359 Subtypes: ABC-type putrescine transporter activity [GO:0015594] Definition: Catalysis of the reaction: ATP + H2O + polyamine(out) = ADP + phosphate + polyamine(in).